{
  "gene": "UniProtKB:P51654",
  "gene_name": "Glypican-3",
  "gene_symbol": "GPC3",
  "term_label": "cell migration",
  "term_id": "GO:0016477"
}